{
  "term_label": "cell-cell adhesion",
  "gene_symbol": "ITGB8",
  "term_id": "GO:0098609",
  "gene_name": "Integrin beta-8",
  "gene": "UniProtKB:P26012"
}